RITS complex localization [GO:0034630] (biological process) Definition: Any process in which a RITS complex is transported to, or maintained in, a specific location. Also known as: RITS complex localisation, establishment and maintenance of RITS complex localization Sources: GOC:mah Relationships: is a type of protein-containing complex localization [GO:0031503]